{
  "term_label": "Unknown molecular function",
  "gene": "UniProtKB:A6NNJ1",
  "gene_name": "Putative protein FAM90A9",
  "gene_symbol": "FAM90A9",
  "term_id": "UNKNOWN:0001"
}